{
  "gene_name": "Late secretory pathway protein AVL9 homolog",
  "gene_symbol": "AVL9",
  "term_id": "GO:0005737",
  "gene": "UniProtKB:Q8NBF6",
  "term_label": "cytoplasm"
}